{
  "term_id": "UNKNOWN:0002",
  "gene_symbol": "NUTM2E",
  "gene_name": "NUT family member 2E",
  "term_label": "Unknown biological process",
  "gene": "UniProtKB:B1AL46"
}